{
  "gene_name": "Dystrophin",
  "term_label": "regulation of muscle system process",
  "gene": "UniProtKB:P11532",
  "gene_symbol": "DMD",
  "term_id": "GO:0090257"
}